{
  "gene_name": "Ribonuclease 3",
  "term_id": "GO:0004525",
  "gene": "UniProtKB:Q9NRR4",
  "term_label": "ribonuclease III activity",
  "gene_symbol": "DROSHA"
}